mitochondrial respiratory chain complex II assembly [GO:0034553] (biological process) Sources: GOC:dgf Definition: The aggregation, arrangement and bonding together of a set of components to form respiratory chain complex II, in the mitochondrial inner membrane. Relationships: is a type of GO:0033108; is a type of respiratory chain complex II assembly [GO:0034552]